{
  "gene_symbol": "KIRREL2",
  "term_label": "cell-cell adhesion",
  "gene_name": "Kin of IRRE-like protein 2",
  "term_id": "GO:0098609",
  "gene": "UniProtKB:Q6UWL6"
}